{
  "gene_symbol": "SREBF2",
  "term_id": "GO:0005634",
  "gene": "UniProtKB:Q12772",
  "term_label": "nucleus",
  "gene_name": "Sterol regulatory element-binding protein 2"
}